{
  "term_label": "regulation of DNA-templated transcription",
  "gene_symbol": "ZNF85",
  "gene": "UniProtKB:Q03923",
  "term_id": "GO:0006355",
  "gene_name": "Zinc finger protein 85"
}